{
  "gene": "UniProtKB:Q96DU7",
  "gene_symbol": "ITPKC",
  "term_id": "GO:0005634",
  "term_label": "nucleus",
  "gene_name": "Inositol-trisphosphate 3-kinase C"
}